{
  "gene_name": "Transmembrane protein 104",
  "gene": "UniProtKB:Q8NE00",
  "term_id": "UNKNOWN:0003",
  "gene_symbol": "TMEM104",
  "term_label": "Unknown cellular component"
}